{
  "gene": "UniProtKB:O15204",
  "term_id": "GO:0006508",
  "gene_symbol": "ADAMDEC1",
  "gene_name": "ADAM DEC1",
  "term_label": "proteolysis"
}